{
  "gene": "UniProtKB:P25440",
  "term_label": "chromatin",
  "term_id": "GO:0000785",
  "gene_name": "Bromodomain-containing protein 2",
  "gene_symbol": "BRD2"
}